{
  "gene": "UniProtKB:Q5SW96",
  "term_id": "UNKNOWN:0001",
  "gene_symbol": "LDLRAP1",
  "gene_name": "Low density lipoprotein receptor adapter protein 1",
  "term_label": "Unknown molecular function"
}